{
  "term_id": "UNKNOWN:0002",
  "gene_symbol": "AVL9",
  "term_label": "Unknown biological process",
  "gene": "UniProtKB:Q8NBF6",
  "gene_name": "Late secretory pathway protein AVL9 homolog"
}